ABC-type vitamin B12 transporter activity [GO:0015420] (molecular function) Also known as: cobalamin porter activity, cobalamin transporter activity, vitamin B12 porter activity, vitamin B12 transporter activity, vitamin B12-transporting ATPase activity, ATP-dependent vitamin B12 transmembrane transporter activity, ATPase-coupled cobalamin transmembrane transporter activity, cobalamin ABC transporter, vitamin B12 ABC transporter activity, ATP-dependent cobalamin transmembrane transporter activity, ATPase-coupled vitamin B12 transmembrane transporter activity, cobalamin-transporting ATPase activity Sources: GOC:pz, RHEA:17873 Relationships: is a type of vitamin transmembrane transporter activity [GO:0090482]; is a type of ABC-type transporter activity [GO:0140359]; is part of cobalamin transport [GO:0015889] Definition: Enables the transfer of a solute or solutes from one side of a membrane to the other according to the reaction: vitamin B12(out) + ATP + H2O = ADP + an vitamin B12(in) + H+ + phosphate. Vitamin B12 is alkylcob(III)alamin.